proline dehydrogenase activity [GO:0004657] (molecular function) Relationships: is a type of oxidoreductase activity, acting on the CH-NH group of donors, quinone or similar compound as acceptor [GO:0016649] Also known as: proline oxidase activity, L-proline dehydrogenase activity Definition: Catalysis of the reaction: L-proline + a quinone = (S)-1-pyrroline-5-carboxylate + a quinol + H+. Sources: RHEA:23784